oxidoreductase activity, acting on the CH-CH group of donors, NAD or NADP as acceptor [GO:0016628] (molecular function) Definition: Catalysis of an oxidation-reduction (redox) reaction in which a CH-CH group acts as a hydrogen or electron donor and reduces NAD or NADP. Sources: EC:1.3.1.- Relationships: is a type of oxidoreductase activity, acting on the CH-CH group of donors [GO:0016627] Subtypes: Delta24(24-1) sterol reductase activity [GO:0000246], GO:0004074, dihydropyrimidine dehydrogenase (NAD+) activity [GO:0004159], dihydroorotate dehydrogenase (NAD+) activity [GO:0004589], prephenate dehydrogenase (NADP+) activity [GO:0004665], 2,3-dihydro-2,3-dihydroxybenzoate dehydrogenase activity [GO:0008667], 2,4-dienoyl-CoA reductase (NADPH) activity [GO:0008670], N-ethylmaleimide reductase activity [GO:0008748], 4-hydroxy-tetrahydrodipicolinate reductase [GO:0008839], GO:0008977, GO:0016156, 12-oxophytodienoate reductase activity [GO:0016629], protochlorophyllide reductase activity [GO:0016630], enoyl-[acyl-carrier-protein] reductase [NAD(P)H] activity [GO:0016631], precorrin-6A reductase activity [GO:0016994], dihydropyrimidine dehydrogenase (NADP+) activity [GO:0017113], 2,3-dihydroxy-2,3-dihydro-phenylpropionate dehydrogenase activity [GO:0018498], 2,5-dichloro-2,5-cyclohexadiene-1,4-diol dehydrogenase activity [GO:0018502], cis-1,2-dihydrobenzene-1,2-diol dehydrogenase activity [GO:0018504], cis-1,2-dihydro-1,2-dihydroxynaphthalene dehydrogenase activity [GO:0018505], maleylacetate reductase activity [GO:0018506], cis-3,4-dihydrophenanthrene-3,4-diol dehydrogenase activity [GO:0018507], cis-2,3-dihydrobiphenyl-2,3-diol dehydrogenase activity [GO:0018509], phloroglucinol reductase activity [GO:0018510], 2,3-dihydroxy-2,3-dihydro-p-cumate dehydrogenase activity [GO:0018511], GO:0018513, pimeloyl-CoA dehydrogenase activity [GO:0018515], GO:0018517, 5,6-dihydroxy-3-methyl-2-oxo-1,2,5,6-tetrahydroquinoline dehydrogenase activity [GO:0018518], cis-dihydroethylcatechol dehydrogenase activity [GO:0018519], GO:0018520, 1,2-dihydroxy-6-methylcyclohexa-3,5-dienecarboxylate dehydrogenase activity [GO:0018521], GO:0019166, 2-alkenal reductase [NAD(P)H] activity [GO:0032440], GO:0033728, GO:0033729, arogenate dehydrogenase [NAD(P)+] activity [GO:0033731], GO:0034824, GO:0034912, enone reductase activity [GO:0035671], 11-hydroxythromboxane B2 dehydrogenase activity [GO:0036133], 12-hydroxyheptadecatrienoic acid synthase activity [GO:0036134], precorrin-2 dehydrogenase activity [GO:0043115], GO:0043786, crotonyl-CoA reductase activity [GO:0043880], GO:0043957, acryloyl-CoA reductase (NADH) activity [GO:0043958], GO:0047114, GO:0047115, GO:0047116, 2-hydroxy-6-oxo-6-phenylhexa-2,4-dienoate reductase activity [GO:0047118], GO:0047120, 15-oxoprostaglandin 13-reductase [NAD(P)+] activity [GO:0047522], 2'-hydroxydaidzein reductase activity [GO:0047525], 2'-hydroxyisoflavone reductase activity [GO:0047526], GO:0047540, GO:0047543, 3-methyleneoxindole reductase activity [GO:0047567], GO:0047598, GO:0047616, alpha-santonin 1,2-reductase activity [GO:0047659], GO:0047703, biochanin-A reductase activity [GO:0047706], cis-2-enoyl-CoA reductase (NADPH) activity [GO:0047774], 2-coumarate reductase activity [GO:0047788], GO:0047794, geissoschizine dehydrogenase activity [GO:0047920], meso-tartrate dehydrogenase activity [GO:0050092], dihydroorotate dehydrogenase (NADP+) activity [GO:0050158], GO:0050343, GO:0050399, zeatin reductase activity [GO:0050472], Delta14-sterol reductase activity [GO:0050613], Delta24-sterol reductase activity [GO:0050614], GO:0050615, (+)-pulegone reductase (NADP+) activity [GO:0052579], curcumin reductase (NADP+) activity [GO:0052849], geranylgeranyl diphosphate reductase activity [GO:0102067], acrolein reductase activity [GO:0102232], 1-penten-3-one reductase activity [GO:0102235], trans-4-hexen-3-one reductase activity [GO:0102236], polyprenol reductase activity [GO:0102389], 2-chloroacrylate reductase activity [GO:0102523], GO:0102758, furaneol oxidoreductase activity [GO:0102978], RNA dihydrouridine synthase activity [GO:0106413], polyprenol dehydrogenase (NAD+) activity [GO:0160196], dolichal reductase (NADPH) activity [GO:0160197], polyprenal reductase activity [GO:0160198]